{
  "term_label": "brain development",
  "term_id": "GO:0007420",
  "gene_symbol": "SOX14",
  "gene_name": "Transcription factor SOX-14",
  "gene": "UniProtKB:O95416"
}